{
  "gene": "UniProtKB:Q9H1Y0",
  "gene_symbol": "ATG5",
  "term_id": "GO:0034045",
  "gene_name": "Autophagy protein 5",
  "term_label": "phagophore assembly site membrane"
}